{
  "term_label": "Unknown cellular component",
  "term_id": "UNKNOWN:0003",
  "gene_symbol": "RASL10A",
  "gene_name": "Ras-like protein family member 10A",
  "gene": "UniProtKB:Q92737"
}